{
  "term_label": "membrane",
  "gene_symbol": "GRINA",
  "term_id": "GO:0016020",
  "gene": "UniProtKB:Q7Z429",
  "gene_name": "Protein lifeguard 1"
}